positive regulation of L-tyrosine import across plasma membrane [GO:1900931] (biological process) Definition: Any process that activates or increases the frequency, rate or extent of L-tyrosine import into the cell. Also known as: positive regulation of L-tyrosine import, up regulation of L-tyrosine import, up-regulation of L-tyrosine import, upregulation of L-tyrosine import, activation of L-tyrosine import, activation of L-tyrosine uptake, positive regulation of L-tyrosine uptake, up regulation of L-tyrosine uptake, up-regulation of L-tyrosine uptake, upregulation of L-tyrosine uptake Relationships: is a type of positive regulation of organic acid transport [GO:0032892]; is_a positive regulation of transmembrane transport [GO:0034764]; is a type of positive regulation of amino acid transport [GO:0051957]; is_a regulation of L-tyrosine import across plasma membrane [GO:1900929]; positively regulates L-tyrosine import across plasma membrane [GO:1903808] Sources: GOC:TermGenie